{
  "term_label": "nucleus",
  "gene": "UniProtKB:P14316",
  "term_id": "GO:0005634",
  "gene_symbol": "IRF2",
  "gene_name": "Interferon regulatory factor 2"
}